{
  "gene_name": "Synaptotagmin-10",
  "gene_symbol": "SYT10",
  "term_label": "plasma membrane",
  "gene": "UniProtKB:Q6XYQ8",
  "term_id": "GO:0005886"
}